{
  "term_id": "GO:0140900",
  "term_label": "chloride:bicarbonate antiporter activity",
  "gene": "UniProtKB:P58743",
  "gene_name": "Prestin",
  "gene_symbol": "SLC26A5"
}